{
  "term_id": "GO:0000978",
  "gene": "UniProtKB:A8MYZ6",
  "term_label": "RNA polymerase II cis-regulatory region sequence-specific DNA binding",
  "gene_symbol": "FOXO6",
  "gene_name": "Forkhead box protein O6"
}